isovaleryl-CoA(4-) biosynthetic process [GO:1902197] (biological process) Definition: The chemical reactions and pathways resulting in the formation of isovaleryl-CoA(4-). References: PMID:11231285 Sources: GOC:TermGenie Also known as: isovaleryl-CoA(4-) anabolism, isovaleryl-CoA(4-) biosynthesis, isovaleryl-CoA(4-) formation, isovaleryl-CoA(4-) synthesis Relationships: is a type of fatty-acyl-CoA biosynthetic process [GO:0046949]